phosphatidylinositol acyl-chain remodeling [GO:0036149] (biological process) Relationships: is a type of phosphatidylinositol metabolic process [GO:0046488] Definition: Remodeling the acyl chains of phosphatidylinositol, through sequential deacylation and re-acylation reactions, to generate phosphatidylinositol containing different types of fatty acid acyl chains. References: PMID:18094042, PMID:18772128 Sources: GOC:mw Also known as: phosphatidylinositol acyl-chain remodelling